{
  "gene_symbol": "IMMP2L",
  "gene": "UniProtKB:Q96T52",
  "term_id": "GO:0006627",
  "gene_name": "Mitochondrial inner membrane protease subunit 2",
  "term_label": "protein processing involved in protein targeting to mitochondrion"
}